{
  "term_id": "GO:0016887",
  "gene_symbol": "CARNS1",
  "gene_name": "Carnosine synthase 1",
  "term_label": "ATP hydrolysis activity",
  "gene": "UniProtKB:A5YM72"
}